{
  "term_id": "UNKNOWN:0001",
  "term_label": "Unknown molecular function",
  "gene_symbol": "OCLN",
  "gene": "UniProtKB:Q16625",
  "gene_name": "Occludin"
}